regulation of o-orsellinic acid biosynthetic process [GO:1900698] (biological process) Definition: Any process that modulates the frequency, rate or extent of o-orsellinic acid biosynthetic process. Sources: GOC:TermGenie, GOC:di Also known as: regulation of o-orsellinic acid anabolism, regulation of o-orsellinic acid biosynthesis, regulation of o-orsellinic acid formation, regulation of o-orsellinic acid synthesis Relationships: is a type of GO:0010565; is a type of regulation of small molecule metabolic process [GO:0062012]; is a type of GO:1900376; regulates o-orsellinic acid biosynthetic process [GO:1900584] Subtypes: negative regulation of o-orsellinic acid biosynthetic process [GO:1900699], positive regulation of o-orsellinic acid biosynthetic process [GO:1900700]